{
  "term_id": "GO:0031647",
  "term_label": "regulation of protein stability",
  "gene_symbol": "USP37",
  "gene": "UniProtKB:Q86T82",
  "gene_name": "Ubiquitin carboxyl-terminal hydrolase 37"
}